positive regulation of artery smooth muscle contraction [GO:1905656] (biological process) Definition: Any process that activates or increases the frequency, rate or extent of artery smooth muscle contraction. Also known as: up regulation of artery smooth muscle contraction, up-regulation of artery smooth muscle contraction, upregulation of artery smooth muscle contraction, activation of artery smooth muscle contraction References: PMID:27389411 Sources: GOC:BHF, GOC:BHF_miRNA, GOC:TermGenie, GOC:rph, GO_REF:0000058 Relationships: is a type of positive regulation of vascular associated smooth muscle contraction [GO:1904695]; is a type of regulation of artery smooth muscle contraction [GO:1905654]; positively regulates GO:0014824